{
  "gene_name": "Leucine-rich repeat and WD repeat-containing protein 1",
  "gene": "UniProtKB:Q9UFC0",
  "gene_symbol": "LRWD1",
  "term_label": "nuclear origin of replication recognition complex",
  "term_id": "GO:0005664"
}